intramembranous bone morphogenesis [GO:1904770] (biological process) Also known as: intramembranous bones morphogenesis, membrane bone morphogenesis Definition: The developmental process by which an intramembranous bone is generated and organized. Relationships: is a type of GO:0060349 References: PMID:26399686 Sources: GOC:TermGenie, GO_REF:0000083